rRNA (adenine-N1-)-methyltransferase activity [GO:0106142] (molecular function) Also known as: 25S rRNA (adenine(645)-N(1))-methyltransferase, 25S rRNA m(1)A(645) methyltransferase Definition: Catalysis of the reaction: S-adenosyl-L-methionine + adenine(645) in 25S rRNA = S-adenosyl-L-homocysteine + N(1)-methyladenine(645) in 25S rRNA. References: PMID:23180764 Sources: EC:2.1.1.287 Relationships: is a type of GO:0016433 Note: The m(1)A modification at position 645 in the large rRNA is highly conserved in eukaryotes.